{
  "gene": "UniProtKB:Q12947",
  "gene_name": "Forkhead box protein F2",
  "term_id": "GO:0000981",
  "gene_symbol": "FOXF2",
  "term_label": "DNA-binding transcription factor activity, RNA polymerase II-specific"
}